{
  "gene_symbol": "TMEM63C",
  "gene": "UniProtKB:Q9P1W3",
  "term_label": "calcium-activated cation channel activity",
  "term_id": "GO:0005227",
  "gene_name": "Calcium permeable stress-gated cation channel 1"
}